angiogenesis [GO:0001525] (biological process) Definition: Blood vessel formation when new vessels emerge from the proliferation of pre-existing blood vessels. Sources: ISBN:0878932453 Also known as: blood vessel formation from pre-existing blood vessels Relationships: is a type of anatomical structure formation involved in morphogenesis [GO:0048646]; is part of GO:0048514 Subtypes: sprouting angiogenesis [GO:0002040], intussusceptive angiogenesis [GO:0002041], GO:0060055, angiogenesis involved in coronary vascular morphogenesis [GO:0060978], GO:0072104 Regulation: negatively regulated by negative regulation of angiogenesis [GO:0016525]; regulated by regulation of angiogenesis [GO:0045765]; positively regulated by GO:0045766